Rad51C-XRCC3 complex [GO:0033065] (cellular component) Also known as: CX3 complex, Rad55-Rad57 complex, Rhp55-Rhp57 complex Definition: A DNA recombinase mediator complex that contains the Rad51 paralogs RAD51C and XRCC3, or orthologs thereof. References: PMID:12427746, PMID:16093548, PMID:17114795 Sources: GOC:mah, GOC:vw Relationships: is a type of DNA recombinase mediator complex [GO:0033061]; is a type of nuclear protein-containing complex [GO:0140513]